{
  "term_id": "UNKNOWN:0001",
  "term_label": "Unknown molecular function",
  "gene": "UniProtKB:B7Z368",
  "gene_symbol": "LINC02881",
  "gene_name": "Uncharacterized protein encoded by LINC02881"
}